{
  "gene": "UniProtKB:Q9HC78",
  "gene_symbol": "ZBTB20",
  "term_id": "GO:0001817",
  "gene_name": "Zinc finger and BTB domain-containing protein 20",
  "term_label": "regulation of cytokine production"
}